cortical microtubule, transverse to long axis [GO:0010005] (cellular component) Sources: ISBN:0943088399 Definition: Arrays of microtubules underlying and connected to the plasma membrane, in the cortical cytosol, oriented mainly with their axes transverse to the long axis of the cell (and root in plants). In plants it influences the direction of cellulose microfibril deposition. Relationships: is a type of GO:0055028